{
  "gene_name": "Olfactory receptor 7C2",
  "gene": "UniProtKB:O60412",
  "term_id": "GO:0007165",
  "term_label": "signal transduction",
  "gene_symbol": "OR7C2"
}